{
  "gene_symbol": "UNC13A",
  "gene_name": "Protein unc-13 homolog A",
  "term_id": "GO:0061789",
  "gene": "UniProtKB:Q9UPW8",
  "term_label": "dense core granule priming"
}